{
  "gene_symbol": "ATG5",
  "gene_name": "Autophagy protein 5",
  "gene": "UniProtKB:Q9H1Y0",
  "term_label": "aggrephagy",
  "term_id": "GO:0035973"
}